positive regulation of muscle hyperplasia [GO:0014739] (biological process) Sources: GOC:mtg_muscle Relationships: is a type of GO:0014738; is a type of positive regulation of muscle adaptation [GO:0014744]; positively regulates muscle hyperplasia [GO:0014900] Definition: Any process that activates or increases the frequency, rate or extent of muscle hyperplasia.